RNA guanosine-cytidine insertion [GO:0070713] (biological process) Also known as: RNA GC insertion Sources: GOC:cb, GOC:mah Definition: The modification of an RNA molecule by insertion of an guanosine-cytidine dinucleotide. Relationships: is a type of RNA dinucleotide insertion [GO:0070707]